pole plasm RNA localization [GO:0007316] (BP) Subtypes: pole plasm mRNA localization [GO:0019094], GO:0019095 Relationships: is a type of RNA localization [GO:0006403]; is part of pole plasm assembly [GO:0007315] Also known as: establishment and maintenance of pole plasm RNA localization, oocyte pole plasm RNA localization, pole plasm RNA localisation Definition: Any process in which RNA is transported to, or maintained in, the oocyte pole plasm. An example of this is found in Drosophila melanogaster. Sources: GOC:ai